Cul7-RING ubiquitin ligase complex [GO:0031467] (cellular component) Relationships: is a type of cullin-RING ubiquitin ligase complex [GO:0031461] References: PMID:15571813, PMID:15688063 Also known as: CDL7 complex, CRL7 complex, SCF7 complex, cullin-RING ligase 7 Definition: A ubiquitin ligase complex in which a cullin from the Cul7 subfamily and a RING domain protein form the catalytic core; substrate specificity is conferred by a Skp1 linker and an F-box protein.